{
  "gene": "UniProtKB:P02549",
  "term_label": "cell junction",
  "term_id": "GO:0030054",
  "gene_symbol": "SPTA1",
  "gene_name": "Spectrin alpha chain, erythrocytic 1"
}